{
  "gene_name": "Synaptogyrin-1",
  "term_id": "GO:0030672",
  "gene_symbol": "SYNGR1",
  "gene": "UniProtKB:O43759",
  "term_label": "synaptic vesicle membrane"
}